skeletal muscle satellite stem cell asymmetric division involved in skeletal muscle regeneration [GO:0014716] (biological process) Sources: GOC:mtg_muscle Note: Occurrence of this process outside of the context of muscle repair is probably very rare, so there is a good case for merging this with the parent class. Relationships: is a type of skeletal muscle satellite stem cell asymmetric division [GO:0014833]; is part of skeletal muscle satellite cell maintenance involved in skeletal muscle regeneration [GO:0014834] Also known as: satellite cell asymmetric division involved in skeletal muscle regeneration Definition: Skeletal muscle satellite cell asymmetric division that occurs during a process in which damaged muscle tissue is being rebuilt.